{
  "gene_symbol": "SLC39A6",
  "gene": "UniProtKB:Q13433",
  "term_id": "GO:0005385",
  "term_label": "zinc ion transmembrane transporter activity",
  "gene_name": "Zinc transporter ZIP6"
}